{
  "term_label": "secretory granule",
  "gene_symbol": "KLK1",
  "gene_name": "Kallikrein-1",
  "term_id": "GO:0030141",
  "gene": "UniProtKB:P06870"
}